mesenchymal cell proliferation involved in prostate gland development [GO:0060781] (biological process) Relationships: is a type of mesenchymal cell proliferation [GO:0010463]; is part of prostate gland development [GO:0030850] Definition: The multiplication or reproduction of mesenchymal cells, resulting in the expansion of a cell population that contributes to the progression of the prostate gland over time. References: PMID:12221011 Sources: GOC:dph Regulation: regulated by regulation of mesenchymal cell proliferation involved in prostate gland development [GO:0060782]